lamellipodium [GO:0030027] (cellular component) Sources: ISBN:0815316194 Relationships: is a type of GO:0120025; is part of cell leading edge [GO:0031252] Subtypes: growth cone lamellipodium [GO:1990761] Definition: A thin sheetlike process extended by the leading edge of a migrating cell or extending cell process; contains a dense meshwork of actin filaments.